conidiophore development [GO:0070787] (biological process) Relationships: is a type of GO:0075259 Regulation: regulated by regulation of conidiophore development [GO:0070793]; negatively regulated by GO:0070794; RO_0002213 by positive regulation of conidiophore development [GO:0070795] Definition: The process whose specific outcome is the progression of the conidiophore over time, from its formation to the mature structure. The conidiophore is a specialized hypha that extends aerially from the growth substrate and bears conidia, or asexual spores. References: PMID:9529886